{
  "term_label": "dynein light intermediate chain binding",
  "term_id": "GO:0051959",
  "gene_symbol": "DNHD1",
  "gene_name": "Dynein heavy chain domain-containing protein 1",
  "gene": "UniProtKB:Q96M86"
}